{
  "gene": "UniProtKB:Q99572",
  "term_label": "cell surface receptor signaling pathway",
  "gene_name": "P2X purinoceptor 7",
  "term_id": "GO:0007166",
  "gene_symbol": "P2RX7"
}